{
  "gene": "UniProtKB:P01562",
  "gene_symbol": "IFNA1",
  "term_label": "natural killer cell activation involved in immune response",
  "gene_name": "Interferon alpha-1_13",
  "term_id": "GO:0002323"
}